negative regulation of mature B cell apoptotic process [GO:0002906] (biological process) Also known as: down regulation of mature B cell apoptosis, down-regulation of mature B cell apoptosis, downregulation of mature B cell apoptosis, inhibition of mature B cell apoptosis, negative regulation of mature B cell apoptosis Definition: Any process that stops, prevents, or reduces the frequency, rate, or extent of mature B cell apoptotic process. Relationships: is a type of negative regulation of B cell apoptotic process [GO:0002903]; is a type of regulation of mature B cell apoptotic process [GO:0002905]; RO_0002212 mature B cell apoptotic process [GO:0002901] Sources: GOC:add, GOC:mtg_apoptosis